cyclin D1-CDK6 complex [GO:0097131] (cellular component) References: PMID:15935619 Sources: GOC:so Relationships: is a type of cyclin-dependent protein kinase holoenzyme complex [GO:0000307] Definition: A protein complex consisting of cyclin D1 and cyclin-dependent kinase 6 (CDK6). Cyclins are characterized by periodicity in protein abundance throughout the cell cycle. Cyclin-dependent kinases represent a family of serine/threonine protein kinases that become active upon binding to a cyclin regulatory partner.